{
  "term_id": "GO:1902476",
  "gene_name": "Solute carrier family 12 member 6",
  "gene_symbol": "SLC12A6",
  "term_label": "chloride transmembrane transport",
  "gene": "UniProtKB:Q9UHW9"
}